{
  "gene_symbol": "LCN8",
  "term_label": "Unknown molecular function",
  "term_id": "UNKNOWN:0001",
  "gene_name": "Epididymal-specific lipocalin-8",
  "gene": "UniProtKB:Q6JVE9"
}